negative regulation of mitotic sister chromatid separation [GO:2000816] (biological process) Definition: Any process that stops, prevents or reduces the frequency, rate or extent of mitotic sister chromatid separation. Sources: GOC:obol Also known as: negative regulation of mitotic sister chromatid resolution, negative regulation of sister chromatid separation during mitosis, negative regulation of chromosome separation during mitosis, negative regulation of mitotic chromosome separation Subtypes: negative regulation of mitotic metaphase/anaphase transition [GO:0045841], negative regulation of mitotic sister chromatid arm separation [GO:1905823] Relationships: is a type of regulation of mitotic sister chromatid separation [GO:0010965]; is a type of negative regulation of mitotic sister chromatid segregation [GO:0033048]; is a type of negative regulation of chromosome separation [GO:1905819]; negatively regulates GO:0051306